{
  "gene": "UniProtKB:P48169",
  "gene_name": "Gamma-aminobutyric acid receptor subunit alpha-4",
  "gene_symbol": "GABRA4",
  "term_label": "GABA-gated chloride ion channel activity",
  "term_id": "GO:0022851"
}